exonuclease activity [GO:0004527] (molecular function) Relationships: is a type of nuclease activity [GO:0004518]; is a type of hydrolase activity, acting on ester bonds [GO:0016788] Definition: Catalysis of the hydrolysis of ester linkages within nucleic acids by removing nucleotide residues from the 3' or 5' end. Also known as: exonuclease IX activity Subtypes: phosphodiesterase I activity [GO:0004528], DNA exonuclease activity [GO:0004529], GO:0004532, 3'-5' exonuclease activity [GO:0008408], GO:0008409 Sources: GOC:mah, ISBN:0198547684